{
  "term_id": "GO:0050728",
  "gene_symbol": "GHRL",
  "term_label": "negative regulation of inflammatory response",
  "gene": "UniProtKB:Q9UBU3",
  "gene_name": "Appetite-regulating hormone"
}